{
  "term_id": "GO:0008285",
  "gene_symbol": "BTG2",
  "gene_name": "Protein BTG2",
  "gene": "UniProtKB:P78543",
  "term_label": "negative regulation of cell population proliferation"
}